negative regulation of chemokine (C-C motif) ligand 5 production [GO:0071650] (biological process) Also known as: negative regulation of CCL5 production, negative regulation of RANTES production, negative regulation of Regulated upon Activation, Normal T-cell Expressed, and Secreted production Relationships: is a type of negative regulation of chemokine production [GO:0032682]; is a type of regulation of chemokine (C-C motif) ligand 5 production [GO:0071649]; negatively regulates chemokine (C-C motif) ligand 5 production [GO:0071609] Definition: Any process that stops, prevents, or reduces the frequency, rate, or extent of production of chemokine (C-C motif) ligand 5. Sources: GOC:mah